green leaf volatile biosynthetic process [GO:0010597] (biological process) References: PMID:17163881 Relationships: is a type of lipoxygenase pathway [GO:0019372] Definition: The chemical reactions and pathways resulting in the formation of volatile molecules emitted from green plants, such as hexenal, hexenol and hexenyl acetate, from linoleic acid or linolenic acid.